{
  "term_label": "glycerol-3-phosphate biosynthetic process",
  "gene_symbol": "GK2",
  "term_id": "GO:0046167",
  "gene_name": "Glycerol kinase 2",
  "gene": "UniProtKB:Q14410"
}